{
  "gene_symbol": "MYPOP",
  "term_id": "GO:0006357",
  "gene": "UniProtKB:Q86VE0",
  "gene_name": "Myb-related transcription factor, partner of profilin",
  "term_label": "regulation of transcription by RNA polymerase II"
}